2-micrometer circle DNA [GO:0005729] (cellular component) Relationships: is a type of extrachromosomal circular DNA [GO:0005727] Definition: A plasmid commonly found in Saccharomyces, inherited in a non-Mendelian manner and often present in 100-400 copies. References: PMID:12073320